{
  "gene_symbol": "GPR155",
  "term_id": "UNKNOWN:0001",
  "gene_name": "Integral membrane protein GPR155",
  "term_label": "Unknown molecular function",
  "gene": "UniProtKB:Q7Z3F1"
}